xanthophyll binding [GO:0051738] (molecular function) Relationships: is a type of isoprenoid binding [GO:0019840]; is a type of pigment binding [GO:0031409] Definition: Binding to xanthophylls, any of several neutral yellow to orange carotenoid pigments containing oxygen. Sources: ISBN:0122146743